nucleosome disassembly/reassembly complex [GO:1990453] (CC) References: PMID:24843044 Sources: GOC:bhm Note: An example of this is EAF7 in Saccharomyces cerevisiae (P53911) in PMID:24843044 (inferred from direct assay). Relationships: is a type of nuclear protein-containing complex [GO:0140513] Definition: A protein complex involved in the disassembly and subsequent reassembly of nucleosomes. It associates with the coding region of transcriptionally active genes where it interacts with the RNA polymerase II and affects its processivity during co-transcriptional RNA processing and maturation. It exists as a functionally independent part of the NuA4 complex. Also known as: eaf5/7/3 complex